{
  "gene_symbol": "MCCD1",
  "gene_name": "Mitochondrial coiled-coil domain protein 1",
  "term_id": "UNKNOWN:0003",
  "term_label": "Unknown cellular component",
  "gene": "UniProtKB:P59942"
}